cellular response to D-galactose [GO:1905378] (biological process) Definition: Any process that results in a change in state or activity of a cell (in terms of movement, secretion, enzyme production, gene expression, etc.) as a result of a D-galactose stimulus. Also known as: cellular response to D-Gal, cellular response to D-galacto-hexose Relationships: is a type of GO:0071331; is a type of GO:1905377 References: PMID:26261574 Sources: GOC:TermGenie, GO_REF:0000071